linoleate 13S-lipoxygenase activity [GO:0016165] (molecular function) Sources: EC:1.13.11.12, GOC:lb Also known as: lipoxygenase activity, carotene oxidase activity, fat oxidase activity, linoleate:oxygen 13-oxidoreductase activity, lionoleate:O2 oxidoreductase activity, lipoperoxidase activity, lipoxidase activity, lipoxydase activity Relationships: is a type of oxidoreductase activity, acting on single donors with incorporation of molecular oxygen, incorporation of two atoms of oxygen [GO:0016702] Definition: Catalysis of the reaction: linoleate + O2 = (9Z,11E)-(13S)-13-hydroperoxyoctadeca-9,11-dienoate.